{
  "gene": "UniProtKB:Q9UBF2",
  "gene_symbol": "COPG2",
  "term_id": "UNKNOWN:0001",
  "term_label": "Unknown molecular function",
  "gene_name": "Coatomer subunit gamma-2"
}